replication fork [GO:0005657] (cellular component) Subtypes: nuclear replication fork [GO:0043596], cytoplasmic replication fork [GO:0043597] Relationships: is a type of cellular anatomical structure [GO:0110165]; BFO_0000050 GO:0005694 Sources: GOC:mah, ISBN:0198547684 Also known as: replication focus Definition: The Y-shaped region of a replicating DNA molecule, resulting from the separation of the DNA strands and in which the synthesis of new strands takes place. Also includes associated protein complexes.